{
  "term_label": "nucleoplasm",
  "gene_symbol": "CMIP",
  "gene": "UniProtKB:Q8IY22",
  "term_id": "GO:0005654",
  "gene_name": "C-Maf-inducing protein"
}